{
  "gene": "UniProtKB:Q9HCM1",
  "term_label": "histone methyltransferase binding",
  "term_id": "GO:1990226",
  "gene_name": "Retroelement silencing factor 1",
  "gene_symbol": "RESF1"
}